{
  "term_label": "non-canonical NF-kappaB signal transduction",
  "gene": "UniProtKB:Q04864",
  "gene_symbol": "REL",
  "gene_name": "Proto-oncogene c-Rel",
  "term_id": "GO:0038061"
}